{
  "gene_symbol": "TMEM268",
  "term_id": "UNKNOWN:0002",
  "gene": "UniProtKB:Q5VZI3",
  "gene_name": "Transmembrane protein 268",
  "term_label": "Unknown biological process"
}